{
  "term_label": "Unknown cellular component",
  "term_id": "UNKNOWN:0003",
  "gene_symbol": "SLC25A25",
  "gene_name": "Mitochondrial adenyl nucleotide antiporter SLC25A25",
  "gene": "UniProtKB:Q6KCM7"
}